{
  "gene_name": "Secretoglobin family 3A member 2",
  "term_id": "GO:0005615",
  "gene_symbol": "SCGB3A2",
  "term_label": "extracellular space",
  "gene": "UniProtKB:Q96PL1"
}